Watasenia-luciferin 2-monooxygenase activity [GO:0050397] (molecular function) Sources: EC:1.13.12.8, MetaCyc:WATASEMIA-LUCIFERIN-2-MONOOXYGENASE-RXN Relationships: is a type of GO:0016703; is a type of GO:0045289 Also known as: luciferase activity, Watasenia-luciferin:oxygen 2-oxidoreductase (decarboxylating), Watasenia-type luciferase activity Definition: Catalysis of the reaction: Watasenia luciferin + O2 = oxidized Watasenia luciferin + CO2 + light.